{
  "term_id": "UNKNOWN:0002",
  "gene_symbol": "A0A8I5QKY2",
  "gene_name": "Uncharacterized protein",
  "term_label": "Unknown biological process",
  "gene": "UniProtKB:A0A8I5QKY2"
}